{
  "gene": "UniProtKB:Q86WW8",
  "gene_symbol": "COA5",
  "term_label": "mitochondrion",
  "gene_name": "Cytochrome c oxidase assembly factor 5",
  "term_id": "GO:0005739"
}